intein-mediated protein splicing [GO:0016539] (biological process) References: PMID:16305544 Sources: GOC:ma Definition: The removal of an internal amino acid sequence (an intein) from a protein during protein maturation; the excision of inteins is precise and the N- and C-terminal exteins are joined by a normal peptide bond. Protein splicing involves 4 nucleophilic displacements by the 3 conserved splice junction residues. Also known as: intein Relationships: is a type of protein splicing [GO:0030908]